{
  "gene_symbol": "HBZ",
  "gene": "UniProtKB:P02008",
  "term_label": "erythrocyte development",
  "term_id": "GO:0048821",
  "gene_name": "Hemoglobin subunit zeta"
}